{
  "term_id": "GO:0000785",
  "gene_name": "Zinc finger MIZ domain-containing protein 2",
  "gene": "UniProtKB:Q8NF64",
  "term_label": "chromatin",
  "gene_symbol": "ZMIZ2"
}